{
  "term_id": "GO:0007088",
  "term_label": "regulation of mitotic nuclear division",
  "gene_name": "Cullin-9",
  "gene": "UniProtKB:Q8IWT3",
  "gene_symbol": "CUL9"
}